inductive cell-cell signaling between paraxial mesoderm and motor neuron precursors [GO:0021916] (biological process) Definition: Short range signaling between cells of the paraxial mesoderm and motor neuron precursors in the spinal cord that specifies the fate of the motor column neuron precursors along the anterior-posterior axis. Relationships: is a type of inductive cell-cell signaling [GO:0031129]; is part of somatic motor neuron fate commitment [GO:0021917] Also known as: inductive cell-cell signalling between paraxial mesoderm and motor neuron precursors References: PMID:11262869 Sources: GOC:cls, GOC:dgh, GOC:dph, GOC:jid, GO_REF:0000021